{
  "gene_symbol": "MAMLD1",
  "term_label": "nuclear body",
  "gene_name": "Mastermind-like domain-containing protein 1",
  "term_id": "GO:0016604",
  "gene": "UniProtKB:Q13495"
}